{
  "gene_name": "Protein phosphatase 1H",
  "term_label": "Unknown biological process",
  "gene": "UniProtKB:Q9ULR3",
  "term_id": "UNKNOWN:0002",
  "gene_symbol": "PPM1H"
}